{
  "term_label": "immunoglobulin mediated immune response",
  "gene_symbol": "IGHV2-70",
  "term_id": "GO:0016064",
  "gene": "UniProtKB:P01814",
  "gene_name": "Immunoglobulin heavy variable 2-70"
}